host cell mitochondrial membrane [GO:0044191] (CC) Subtypes: host cell mitochondrial inner membrane [GO:0044192], host cell mitochondrial outer membrane [GO:0044193] Definition: Either of the lipid bilayers that surround the host cell mitochondrion and form the host cell mitochondrial envelope. Sources: GOC:jl Relationships: is a type of host cell membrane [GO:0033644]; is part of host cell mitochondrial envelope [GO:0044190]